{
  "term_id": "GO:0007188",
  "term_label": "adenylate cyclase-modulating G protein-coupled receptor signaling pathway",
  "gene_name": "Guanine nucleotide-binding protein G(z) subunit alpha",
  "gene_symbol": "GNAZ",
  "gene": "UniProtKB:P19086"
}